{
  "term_label": "spliceosomal snRNP assembly",
  "gene_name": "Small nuclear ribonucleoprotein Sm D2",
  "gene": "UniProtKB:P62316",
  "gene_symbol": "SNRPD2",
  "term_id": "GO:0000387"
}